{
  "term_label": "response to steroid hormone",
  "gene_name": "Membrane progestin receptor beta",
  "term_id": "GO:0048545",
  "gene": "UniProtKB:Q8TEZ7",
  "gene_symbol": "PAQR8"
}